{
  "term_label": "Unknown molecular function",
  "term_id": "UNKNOWN:0001",
  "gene_symbol": "EIPR1",
  "gene": "UniProtKB:Q53HC9",
  "gene_name": "EARP and GARP complex-interacting protein 1"
}